regulation of cap-independent translational initiation [GO:1903677] (biological process) Definition: Any process that modulates the frequency, rate or extent of cap-independent translational initiation. Sources: GOC:PARL, GOC:TermGenie, GOC:bf, GO_REF:0000058 Relationships: is a type of regulation of cytoplasmic translational initiation [GO:1904688]; regulates GO:0002190 Subtypes: negative regulation of cap-independent translational initiation [GO:1903678], positive regulation of cap-independent translational initiation [GO:1903679]